{
  "gene_name": "Spectrin beta chain, erythrocytic",
  "gene": "UniProtKB:P11277",
  "term_label": "cortical actin cytoskeleton",
  "gene_symbol": "SPTB",
  "term_id": "GO:0030864"
}